hemoglobin complex [GO:0005833] (cellular component) Also known as: haemoglobin complex Definition: An iron-containing, oxygen carrying complex. In vertebrates it is made up of two pairs of associated globin polypeptide chains, each chain carrying a noncovalently bound heme prosthetic group. Sources: GOC:jl, ISBN:0198506732 Relationships: is a type of protein-containing complex [GO:0032991]; is part of cytosol [GO:0005829]